{
  "gene_symbol": "PABPC3",
  "gene_name": "Polyadenylate-binding protein 3",
  "term_label": "nucleus",
  "gene": "UniProtKB:Q9H361",
  "term_id": "GO:0005634"
}